trigeminal ganglion morphogenesis [GO:0061556] (biological process) Also known as: trigeminal ganglia morphogenesis Sources: GOC:dph Definition: The process in which the anatomical structure of a trigeminal ganglion is generated and organized. Relationships: is a type of cranial ganglion morphogenesis [GO:0061559]; is part of trigeminal nerve morphogenesis [GO:0021636]; is part of GO:0061551